transition metal ion transmembrane transporter activity [GO:0046915] (molecular function) Sources: ISBN:0198506732 Definition: Enables the transfer of transition metal ions from one side of a membrane to the other. A transition metal is an element whose atom has an incomplete d-subshell of extranuclear electrons, or which gives rise to a cation or cations with an incomplete d-subshell. Transition metals often have more than one valency state. Biologically relevant transition metals include vanadium, manganese, iron, copper, cobalt, nickel, molybdenum and silver. Subtypes: GO:0005375, iron ion transmembrane transporter activity [GO:0005381], manganese ion transmembrane transporter activity [GO:0005384], zinc ion transmembrane transporter activity [GO:0005385], silver ion transmembrane transporter activity [GO:0015080], cadmium ion transmembrane transporter activity [GO:0015086], GO:0015087, GO:0015097, nickel cation transmembrane transporter activity [GO:0015099], vanadium ion transmembrane transporter activity [GO:0015100], molybdenum ion transmembrane transporter activity [GO:0042888] Relationships: is a type of GO:0046873; is part of GO:0000041